{
  "gene_name": "Protein phosphatase Slingshot homolog 1",
  "term_label": "actin cytoskeleton organization",
  "gene": "UniProtKB:Q8WYL5",
  "gene_symbol": "SSH1",
  "term_id": "GO:0030036"
}